{
  "gene_symbol": "NPM2",
  "gene_name": "Nucleoplasmin-2",
  "term_id": "GO:0045740",
  "term_label": "positive regulation of DNA replication",
  "gene": "UniProtKB:Q86SE8"
}